neuron migration involved in dendrite retrograde extension [GO:0003395] (biological process) Sources: GOC:ascb_2009, GOC:dph, GOC:tb Relationships: is a type of neuron migration involved in retrograde extension [GO:0003393]; is part of dendrite development by retrograde extension [GO:0003390] Definition: The directed, self-propelled movement of a neuron that contributes to the process of retrograde extension of a dendrite. Subtypes: neuron migration involved in amphid sensory organ dendrite retrograde extension [GO:0003397]